{
  "term_label": "neuron projection",
  "term_id": "GO:0043005",
  "gene_name": "Neuropeptide Y receptor type 5",
  "gene": "UniProtKB:Q15761",
  "gene_symbol": "NPY5R"
}